{
  "gene_name": "Myelin protein zero-like protein 3",
  "gene_symbol": "MPZL3",
  "term_id": "UNKNOWN:0002",
  "gene": "UniProtKB:Q6UWV2",
  "term_label": "Unknown biological process"
}